epidermal growth factor catabolic process [GO:0007174] (biological process) Also known as: EGF breakdown, EGF catabolism, epidermal growth factor breakdown, epidermal growth factor catabolism, EGF receptor ligand processing, epidermal growth factor ligand processing, intracellular EGF processing, receptor-mediated EGF processing Note: This term describes the breakdown of epidermal growth factor within the cell, following internalization. For proteolysis events that result in the maturation of an epidermal growth factor receptor ligand, see 'epidermal growth factor receptor ligand maturation ; GO:'. References: PMID:2985587 Sources: GOC:bf, GOC:signaling Relationships: is a type of protein catabolic process [GO:0030163]; is a type of negative regulation of epidermal growth factor receptor signaling pathway [GO:0042059] Definition: The chemical reactions and pathways resulting in the breakdown of epidermal growth factor (EGF), following internalization of the receptor-bound ligand into the signal-receiving cell. Full breakdown of epidermal growth factor results in a ligand that is unable to bind and activate its receptor.